{
  "gene_symbol": "RRN3",
  "term_label": "nucleus",
  "gene": "UniProtKB:Q9NYV6",
  "term_id": "GO:0005634",
  "gene_name": "RNA polymerase I-specific transcription initiation factor RRN3"
}